positive regulation of purine nucleotide metabolic process [GO:1900544] (biological process) Sources: GOC:TermGenie Definition: Any process that activates or increases the frequency, rate or extent of purine nucleotide metabolic process. Also known as: positive regulation of purine nucleotide metabolism, up regulation of purine nucleotide metabolic process, up regulation of purine nucleotide metabolism, up-regulation of purine nucleotide metabolic process, up-regulation of purine nucleotide metabolism, upregulation of purine nucleotide metabolic process, upregulation of purine nucleotide metabolism, activation of purine metabolic process, activation of purine metabolism, activation of purine nucleotide metabolic process, activation of purine nucleotide metabolism, positive regulation of purine metabolic process, positive regulation of purine metabolism, up regulation of purine metabolic process, up regulation of purine metabolism, up-regulation of purine metabolic process, up-regulation of purine metabolism, upregulation of purine metabolic process, upregulation of purine metabolism Relationships: is a type of GO:0045981; is a type of regulation of purine nucleotide metabolic process [GO:1900542]; positively regulates purine nucleotide metabolic process [GO:0006163] Subtypes: positive regulation of purine nucleotide catabolic process [GO:0033123], positive regulation of purine nucleotide biosynthetic process [GO:1900373], positive regulation of NAD metabolic process [GO:1902690], positive regulation of ATP metabolic process [GO:1903580], GO:1905857